{
  "term_label": "progesterone receptor signaling pathway",
  "term_id": "GO:0050847",
  "gene_symbol": "SRC",
  "gene_name": "Proto-oncogene tyrosine-protein kinase Src",
  "gene": "UniProtKB:P12931"
}